{
  "gene": "UniProtKB:Q14517",
  "term_id": "GO:0005886",
  "term_label": "plasma membrane",
  "gene_name": "Protocadherin Fat 1",
  "gene_symbol": "FAT1"
}